{
  "gene": "UniProtKB:P09630",
  "gene_symbol": "HOXC6",
  "term_id": "GO:0000978",
  "gene_name": "Homeobox protein Hox-C6",
  "term_label": "RNA polymerase II cis-regulatory region sequence-specific DNA binding"
}